positive regulation of fibroblast chemotaxis [GO:1905212] (BP) Definition: Any process that activates or increases the frequency, rate or extent of fibroblast chemotaxis. Also known as: up regulation of fibroblast chemotaxis, up-regulation of fibroblast chemotaxis, upregulation of fibroblast chemotaxis, activation of fibroblast chemotaxis Relationships: is a type of positive regulation of cell migration [GO:0030335]; is a type of GO:0050921; is a type of regulation of fibroblast chemotaxis [GO:1905210]; positively regulates GO:1990956 References: PMID:8760137 Sources: GOC:TermGenie, GO_REF:0000058